{
  "gene_symbol": "PLK1",
  "gene": "UniProtKB:P53350",
  "term_id": "GO:0005813",
  "term_label": "centrosome",
  "gene_name": "Serine_threonine-protein kinase PLK1"
}